{
  "gene": "UniProtKB:Q8WUF8",
  "gene_symbol": "ARB2A",
  "term_id": "GO:0035197",
  "gene_name": "Cotranscriptional regulator FAM172A",
  "term_label": "siRNA binding"
}